{
  "term_label": "Unknown biological process",
  "term_id": "UNKNOWN:0002",
  "gene": "UniProtKB:Q16864",
  "gene_symbol": "ATP6V1F",
  "gene_name": "V-type proton ATPase subunit F"
}